{
  "gene_symbol": "LIG1",
  "term_label": "DNA ligase (ATP) activity",
  "gene": "UniProtKB:P18858",
  "gene_name": "DNA ligase 1",
  "term_id": "GO:0003910"
}